{
  "gene_symbol": "MEIS3P2",
  "gene_name": "Putative homeobox protein Meis3-like 2",
  "gene": "UniProtKB:A8K0S8",
  "term_id": "GO:0001525",
  "term_label": "angiogenesis"
}